{
  "gene_name": "Tubulin alpha-4A chain",
  "term_id": "GO:0005737",
  "gene_symbol": "TUBA4A",
  "term_label": "cytoplasm",
  "gene": "UniProtKB:P68366"
}